{
  "gene": "UniProtKB:P23297",
  "gene_name": "Protein S100-A1",
  "term_id": "GO:0005737",
  "term_label": "cytoplasm",
  "gene_symbol": "S100A1"
}